{
  "term_id": "GO:0032426",
  "term_label": "stereocilium tip",
  "gene_name": "Myosin-IIIb",
  "gene": "UniProtKB:Q8WXR4",
  "gene_symbol": "MYO3B"
}